cerebellar molecular layer morphogenesis [GO:0021687] (biological process) Relationships: is a type of anatomical structure morphogenesis [GO:0009653]; is part of cerebellar molecular layer development [GO:0021679]; is part of GO:0021696 Sources: GOC:cls, GOC:dgh, GOC:dph, GOC:jid, GO_REF:0000021 Definition: The process in which the anatomical structure of the cerebellar molecular layer is generated and organized. The molecular layer is the outermost layer of the cerebellar cortex. It contains the parallel fibers of the granule cells, interneurons such as stellate and basket cells, and the dendrites of the underlying Purkinje cells.